{
  "gene_name": "Retinoic acid receptor RXR-beta",
  "term_label": "RNA polymerase II transcription regulator complex",
  "gene_symbol": "RXRB",
  "term_id": "GO:0090575",
  "gene": "UniProtKB:P28702"
}